{
  "gene": "UniProtKB:Q9Y2J8",
  "gene_symbol": "PADI2",
  "gene_name": "Protein-arginine deiminase type-2",
  "term_id": "GO:0005634",
  "term_label": "nucleus"
}